{
  "gene_name": "Putative KHDC1-like protein",
  "gene_symbol": "KHDC1L",
  "term_label": "RNA binding",
  "gene": "UniProtKB:Q5JSQ8",
  "term_id": "GO:0003723"
}